cis-2-enoyl-CoA reductase (NADPH) activity [GO:0047774] (molecular function) Sources: EC:1.3.1.37 Definition: Catalysis of the reaction: acyl-CoA + NADP+ = cis-2,3-dehydroacyl-CoA + NADPH. Relationships: is a type of oxidoreductase activity, acting on the CH-CH group of donors, NAD or NADP as acceptor [GO:0016628] Also known as: NADPH-dependent cis-enoyl-CoA reductase activity, acyl-CoA:NADP+ cis-2-oxidoreductase activity, cis-2-enoyl-coenzyme A reductase activity, reductase, cis-2-enoyl coenzyme A